{
  "gene_name": "Triosephosphate isomerase",
  "term_label": "glyceraldehyde-3-phosphate biosynthetic process",
  "gene_symbol": "TPI1",
  "term_id": "GO:0046166",
  "gene": "UniProtKB:P60174"
}